{
  "term_label": "plasma membrane",
  "gene_symbol": "OR52B2",
  "gene_name": "Olfactory receptor 52B2",
  "gene": "UniProtKB:Q96RD2",
  "term_id": "GO:0005886"
}